{
  "term_id": "GO:0015179",
  "term_label": "L-amino acid transmembrane transporter activity",
  "gene_name": "Y+L amino acid transporter 2",
  "gene_symbol": "SLC7A6",
  "gene": "UniProtKB:Q92536"
}